{
  "term_id": "UNKNOWN:0003",
  "gene": "UniProtKB:Q8TDI8",
  "gene_name": "Transmembrane channel-like protein 1",
  "gene_symbol": "TMC1",
  "term_label": "Unknown cellular component"
}